N5,N10-methenyltetrahydromethanopterin hydrogenase activity [GO:0047068] (MF) Definition: Catalysis of the reaction: 5,10-methenyl-5,6,7,8-tetrahydromethanopterin + H(2) = 5,10-methylenetetrahydromethanopterin + H+. Relationships: is a type of oxidoreductase activity, acting on hydrogen as donor, with other known acceptors [GO:0046995] Also known as: N5,N10-methylenetetrahydromethanopterin dehydrogenase activity, 5,10-methenyltetrahydromethanopterin hydrogenase activity, H(2)-dependent methylene-H(4)MPT dehydrogenase activity, H(2)-forming N(5),N(10)-methylenetetrahydromethanopterin dehydrogenase activity, H2-dependent methylene-H4MPT dehydrogenase activity, H2-forming N5,N10-methylenetetrahydromethanopterin dehydrogenase activity, N(5),N(10)-methenyltetrahydromethanopterin hydrogenase activity, hydrogen:5,10-methenyltetrahydromethanopterin oxidoreductase activity, hydrogen:N(5),N(10)-methenyltetrahydromethanopterin oxidoreductase activity, hydrogen:N5,N10-methenyltetrahydromethanopterin oxidoreductase activity, nonmetal hydrogenase activity Sources: EC:1.12.98.2, RHEA:20017